{
  "term_label": "DNA-binding transcription factor activity, RNA polymerase II-specific",
  "gene_symbol": "KLF7",
  "gene_name": "Krueppel-like factor 7",
  "gene": "UniProtKB:O75840",
  "term_id": "GO:0000981"
}